{
  "term_label": "pyruvate dehydrogenase (acetyl-transferring) kinase activity",
  "term_id": "GO:0004740",
  "gene": "UniProtKB:Q15118",
  "gene_name": "[Pyruvate dehydrogenase (acetyl-transferring)] kinase isozyme 1, mitochondrial",
  "gene_symbol": "PDK1"
}